{
  "gene_name": "Sodium-dependent phosphate transport protein 2A",
  "term_label": "sodium-dependent phosphate transport",
  "gene": "UniProtKB:Q06495",
  "term_id": "GO:0044341",
  "gene_symbol": "SLC34A1"
}